{
  "gene_symbol": "FN1",
  "gene": "UniProtKB:P02751",
  "gene_name": "Fibronectin",
  "term_label": "heart development",
  "term_id": "GO:0007507"
}